arginine:ornithine antiporter activity [GO:0043858] (molecular function) Definition: Catalysis of the reaction: arginine(out) + ornithine(in) = arginine(in) + ornithine(out). References: PMID:17110979 Sources: GOC:jl, RHEA:34991 Also known as: arginine-ornithine antiporter activity, arginine/ornithine antiporter activity, ArcD Relationships: is a type of GO:0015171; is a type of antiporter activity [GO:0015297]; is_a carboxylic acid transmembrane transporter activity [GO:0046943]